regulation of cell differentiation [GO:0045595] (biological process) Sources: GOC:go_curators Subtypes: regulation of epithelial to mesenchymal transition [GO:0010717], regulation of macrophage derived foam cell differentiation [GO:0010743], regulation of epithelial cell differentiation [GO:0030856], regulation of sorocarp stalk cell differentiation [GO:0031285], regulation of chondrocyte differentiation [GO:0032330], GO:0045596, positive regulation of cell differentiation [GO:0045597], regulation of fat cell differentiation [GO:0045598], regulation of hemocyte differentiation [GO:0045610], regulation of myoblast differentiation [GO:0045661], regulation of neuron differentiation [GO:0045664], regulation of osteoblast differentiation [GO:0045667], regulation of glial cell differentiation [GO:0045685], regulation of antipodal cell differentiation [GO:0045688], regulation of embryo sac central cell differentiation [GO:0045691], regulation of embryo sac egg cell differentiation [GO:0045694], regulation of synergid differentiation [GO:0045697], regulation of timing of cell differentiation [GO:0048505], regulation of pigment cell differentiation [GO:0050932], regulation of muscle cell differentiation [GO:0051147], regulation of cell development [GO:0060284], regulation of cell differentiation involved in tissue homeostasis [GO:0060786], regulation of cell differentiation involved in embryonic placenta development [GO:0060800], regulation of cardiac endothelial to mesenchymal transition [GO:0061999], regulation of trichome patterning [GO:1900032], regulation of sorocarp spore cell differentiation [GO:1901261], regulation of hematopoietic progenitor cell differentiation [GO:1901532], GO:1903224, regulation of transdifferentiation [GO:1903618], regulation of plant epidermal cell differentiation [GO:1903888], regulation of sclerenchyma cell differentiation [GO:1904368], regulation of myofibroblast differentiation [GO:1904760], regulation of cardiocyte differentiation [GO:1905207], regulation of mesodermal cell differentiation [GO:1905770], GO:1905915, regulation of trichome morphogenesis [GO:2000039], GO:2000592, regulation of stem cell differentiation [GO:2000736], regulation of skeletal muscle cell differentiation [GO:2001014], GO:2001049, regulation of vasculogenesis [GO:2001212] Relationships: is a type of GO:0050793; is a type of regulation of cellular process [GO:0050794]; RO_0002211 cell differentiation [GO:0030154] Definition: Any process that modulates the frequency, rate or extent of cell differentiation, the process in which relatively unspecialized cells acquire specialized structural and functional features.